{
  "gene_symbol": "FSIP2",
  "gene_name": "Fibrous sheath-interacting protein 2",
  "term_label": "Unknown cellular component",
  "gene": "UniProtKB:Q5CZC0",
  "term_id": "UNKNOWN:0003"
}